serine-type peptidase complex [GO:1905286] (cellular component) Definition: A protein complex which is capable of serine-type peptidase activity. Also known as: Factor VII - TF complex References: PMID:18640965 Sources: GOC:TermGenie, GOC:bhm, GO_REF:0000088 Note: An example of this is F7 in human (P08709) in PMID:18640965 (inferred from direct assay). Subtypes: serine-type endopeptidase complex [GO:1905370] Relationships: is_a peptidase complex [GO:1905368]